{
  "gene": "UniProtKB:P29353",
  "gene_name": "SHC-transforming protein 1",
  "term_label": "insulin receptor signaling pathway",
  "gene_symbol": "SHC1",
  "term_id": "GO:0008286"
}